{
  "term_id": "GO:0000082",
  "term_label": "G1/S transition of mitotic cell cycle",
  "gene_name": "Cyclin-P",
  "gene": "UniProtKB:Q9H8S5",
  "gene_symbol": "CCNP"
}